structural constituent of nuclear pore [GO:0017056] (molecular function) Note: Note that this term is meant to be used for nuclear pore proteins. For importins and exportins, consider 'nuclear import signal receptor activity' or 'nuclear export signal receptor activity', respectively. Relationships: is a type of structural molecule activity [GO:0005198]; is part of nucleocytoplasmic transport [GO:0006913]; BFO_0000066 nuclear pore [GO:0005643] References: PMID:25802992 Sources: GOC:mah Also known as: nucleocytoplasmic transporter activity, nuclear pore activity Definition: The action of a molecule that contributes to the structural integrity of the nuclear pore complex, a protein-lined channel in the nuclear envelope that allows the transfer of macromolecules.